{
  "term_id": "GO:0050810",
  "term_label": "regulation of steroid biosynthetic process",
  "gene_symbol": "STAR",
  "gene": "UniProtKB:P49675",
  "gene_name": "Steroidogenic acute regulatory protein, mitochondrial"
}